{
  "term_label": "cytoplasm",
  "term_id": "GO:0005737",
  "gene_name": "Cyclin-J",
  "gene_symbol": "CCNJ",
  "gene": "UniProtKB:Q5T5M9"
}